negative regulation of mitochondrial mRNA catabolic process [GO:1905638] (biological process) References: PMID:27122350 Sources: GOC:TermGenie, GO_REF:0000058 Definition: Any process that stops, prevents or reduces the frequency, rate or extent of mitochondrial mRNA catabolic process. Also known as: down regulation of mitochondrial mRNA catabolic process, down-regulation of mitochondrial mRNA catabolic process, downregulation of mitochondrial mRNA catabolic process, inhibition of mitochondrial mRNA catabolic process Relationships: is_a GO:0000961; is a type of negative regulation of mRNA catabolic process [GO:1902373]; is a type of GO:1905637; negatively regulates GO:0000958